righting reflex [GO:0060013] (biological process) Definition: A reflex process in which an animal immediately tries to turn over after being placed in a supine position. References: PMID:8635460 Sources: GOC:dph Also known as: righting response Relationships: is a type of reflex [GO:0060004]